{
  "gene_symbol": "LSMEM2",
  "gene": "UniProtKB:Q8N112",
  "term_id": "UNKNOWN:0001",
  "term_label": "Unknown molecular function",
  "gene_name": "Leucine-rich single-pass membrane protein 2"
}